{
  "gene": "UniProtKB:Q92772",
  "gene_name": "Cyclin-dependent kinase-like 2",
  "term_label": "nucleus",
  "gene_symbol": "CDKL2",
  "term_id": "GO:0005634"
}